{
  "gene_name": "Cullin-4A",
  "term_id": "GO:0006974",
  "term_label": "DNA damage response",
  "gene_symbol": "CUL4A",
  "gene": "UniProtKB:Q13619"
}